{
  "gene_symbol": "NOD1",
  "gene_name": "Nucleotide-binding oligomerization domain-containing protein 1",
  "term_label": "pattern recognition receptor activity",
  "term_id": "GO:0038187",
  "gene": "UniProtKB:Q9Y239"
}